mitochondrial FAD transmembrane transport [GO:1990548] (biological process) Definition: The process in which FAD is transported across a mitochondrial membrane, into or out of the mitochondrion. References: PMID:14555654 Relationships: is a type of FAD transmembrane transport [GO:0035350]